{
  "gene_symbol": "ESF1",
  "term_id": "UNKNOWN:0003",
  "gene": "UniProtKB:Q9H501",
  "term_label": "Unknown cellular component",
  "gene_name": "ESF1 homolog"
}